{
  "gene_name": "SLIT-ROBO Rho GTPase-activating protein 2B",
  "gene": "UniProtKB:P0DMP2",
  "term_id": "GO:0030336",
  "gene_symbol": "SRGAP2B",
  "term_label": "negative regulation of cell migration"
}